{
  "term_label": "metalloendopeptidase activity",
  "gene": "UniProtKB:A6NFA1",
  "gene_symbol": "TRABD2B",
  "term_id": "GO:0004222",
  "gene_name": "Metalloprotease TIKI2"
}